{
  "gene_symbol": "MSI1",
  "term_label": "cytoplasm",
  "gene_name": "RNA-binding protein Musashi homolog 1",
  "term_id": "GO:0005737",
  "gene": "UniProtKB:O43347"
}